{
  "gene_name": "KN motif and ankyrin repeat domain-containing protein 2",
  "gene_symbol": "KANK2",
  "term_id": "GO:0070563",
  "term_label": "negative regulation of vitamin D receptor signaling pathway",
  "gene": "UniProtKB:Q63ZY3"
}